{
  "gene_name": "Transmembrane protein 216",
  "gene": "UniProtKB:Q9P0N5",
  "term_label": "Unknown molecular function",
  "gene_symbol": "TMEM216",
  "term_id": "UNKNOWN:0001"
}